{
  "term_id": "UNKNOWN:0003",
  "gene_symbol": "CIAO2A",
  "term_label": "Unknown cellular component",
  "gene_name": "Cytosolic iron-sulfur assembly component 2A",
  "gene": "UniProtKB:Q9H5X1"
}